{
  "gene_symbol": "C4orf51",
  "gene_name": "Uncharacterized protein C4orf51",
  "gene": "UniProtKB:C9J302",
  "term_label": "Unknown cellular component",
  "term_id": "UNKNOWN:0003"
}